{
  "gene": "UniProtKB:Q9GZU7",
  "gene_name": "Carboxy-terminal domain RNA polymerase II polypeptide A small phosphatase 1",
  "term_label": "Unknown cellular component",
  "term_id": "UNKNOWN:0003",
  "gene_symbol": "CTDSP1"
}